{
  "term_label": "monocarboxylic acid transmembrane transporter activity",
  "gene_name": "Monocarboxylate transporter 13",
  "gene_symbol": "SLC16A13",
  "term_id": "GO:0008028",
  "gene": "UniProtKB:Q7RTY0"
}